host cell lipid droplet [GO:0044186] (cellular component) Definition: Any particle of coalesced lipids in the cytoplasm of a host cell. May include associated proteins. Also known as: host cell lipid adiposome, host cell lipid body, host cell lipid particle Relationships: is a type of host cell cytoplasm part [GO:0033655] Sources: GOC:jl